{
  "gene": "UniProtKB:Q8IYI6",
  "term_label": "intracellular protein localization",
  "term_id": "GO:0008104",
  "gene_name": "Exocyst complex component 8",
  "gene_symbol": "EXOC8"
}